{
  "gene_symbol": "PHF2",
  "term_id": "UNKNOWN:0003",
  "gene": "UniProtKB:O75151",
  "gene_name": "Lysine-specific demethylase PHF2",
  "term_label": "Unknown cellular component"
}